box C/D sno(s)RNA 5'-end processing [GO:0106410] (biological process) Relationships: is a type of box C/D sno(s)RNA processing [GO:0034963]; is a type of snoRNA 2,2,7-trimethylguanosine (TMG) capping [GO:0180031] Definition: Any process involved in forming the mature 5' end of a box C/D RNA molecule. References: PMID:34352089